{
  "gene": "UniProtKB:P48547",
  "gene_symbol": "KCNC1",
  "term_id": "GO:0042734",
  "term_label": "presynaptic membrane",
  "gene_name": "Potassium voltage-gated channel subfamily C member 1"
}